{
  "term_id": "UNKNOWN:0002",
  "gene_name": "Olfactory receptor 14K1",
  "gene": "UniProtKB:Q8NGZ2",
  "gene_symbol": "OR14K1",
  "term_label": "Unknown biological process"
}